{
  "gene": "UniProtKB:O60921",
  "term_id": "GO:0044778",
  "term_label": "meiotic DNA integrity checkpoint signaling",
  "gene_symbol": "HUS1",
  "gene_name": "Checkpoint protein HUS1"
}